{
  "term_id": "GO:0000978",
  "gene_name": "Zinc finger protein 575",
  "gene_symbol": "ZNF575",
  "gene": "UniProtKB:Q86XF7",
  "term_label": "RNA polymerase II cis-regulatory region sequence-specific DNA binding"
}